regulation of immunoglobulin production in mucosal tissue [GO:2000557] (biological process) Definition: Any process that modulates the frequency, rate or extent of immunoglobulin production in mucosal tissue. Relationships: is a type of regulation of immunoglobulin production [GO:0002637]; is a type of GO:0002889; regulates GO:0002426 Also known as: regulation of antibody production in mucosal tissue Sources: GOC:obol Subtypes: positive regulation of immunoglobulin production in mucosal tissue [GO:2000558]